regulation of urea catabolic process [GO:0034254] (biological process) Also known as: regulation of urea breakdown, regulation of urea catabolism, regulation of urea degradation Subtypes: GO:1901713, GO:1901714 Sources: GOC:mah Definition: Any process that modulates the frequency, rate or extent of the chemical reactions and pathways resulting in the breakdown of urea. Relationships: is a type of regulation of amide catabolic process [GO:0034251]; is a type of GO:0062012; is a type of regulation of nitrogen cycle metabolic process [GO:1903314]; regulates urea catabolic process [GO:0043419]